{
  "term_id": "GO:0007131",
  "gene_symbol": "RAD51C",
  "gene_name": "DNA repair protein RAD51 homolog 3",
  "gene": "UniProtKB:O43502",
  "term_label": "reciprocal meiotic recombination"
}